{
  "gene_symbol": "SLC30A8",
  "term_label": "plasma membrane",
  "gene_name": "Proton-coupled zinc antiporter SLC30A8",
  "term_id": "GO:0005886",
  "gene": "UniProtKB:Q8IWU4"
}